{
  "gene_symbol": "TLR1",
  "term_label": "cellular response to triacyl bacterial lipopeptide",
  "gene_name": "Toll-like receptor 1",
  "gene": "UniProtKB:Q15399",
  "term_id": "GO:0071727"
}